{
  "gene_name": "Platelet factor 4 variant",
  "term_id": "GO:0030593",
  "gene_symbol": "PF4V1",
  "gene": "UniProtKB:P10720",
  "term_label": "neutrophil chemotaxis"
}